N-acetylglucosamine 6-O-sulfotransferase activity [GO:0001517] (molecular function) Sources: GOC:ai, GOC:hjd Definition: Catalysis of the reaction: 3'-phosphoadenosine 5'-phosphosulfate + N-acetyl-D-glucosamine = adenosine 3',5'-bisphosphate + N-acetyl-D-glucosamine 6-sulfate. Relationships: is a type of sulfotransferase activity [GO:0008146] Also known as: N-acetylglucosamine 6-O-sulphotransferase activity